{
  "gene_name": "Large ribosomal subunit protein mL66",
  "gene": "UniProtKB:Q9NVS2",
  "term_label": "mitochondrial small ribosomal subunit",
  "gene_symbol": "MRPS18A",
  "term_id": "GO:0005763"
}